{
  "term_id": "GO:0005509",
  "gene": "UniProtKB:Q9BUY7",
  "term_label": "calcium ion binding",
  "gene_symbol": "EFCAB11",
  "gene_name": "EF-hand calcium-binding domain-containing protein 11"
}